{
  "term_label": "Unknown biological process",
  "gene": "UniProtKB:Q53T59",
  "gene_name": "HCLS1-binding protein 3",
  "gene_symbol": "HS1BP3",
  "term_id": "UNKNOWN:0002"
}